regulation of tensidol A biosynthetic process [GO:1900707] (biological process) Relationships: is a type of regulation of ketone biosynthetic process [GO:0010566]; is a type of regulation of amide metabolic process [GO:0034248]; is a type of regulation of secondary metabolite biosynthetic process [GO:1900376]; regulates tensidol A biosynthetic process [GO:1900605] Definition: Any process that modulates the frequency, rate or extent of tensidol A biosynthetic process. Also known as: regulation of tensidol A anabolism, regulation of tensidol A biosynthesis, regulation of tensidol A formation, regulation of tensidol A synthesis Subtypes: GO:1900708, positive regulation of tensidol A biosynthetic process [GO:1900709] Sources: GOC:TermGenie, GOC:di